{
  "term_label": "vesicle-mediated transport",
  "gene": "UniProtKB:Q9BW83",
  "term_id": "GO:0016192",
  "gene_name": "Intraflagellar transport protein 27 homolog",
  "gene_symbol": "IFT27"
}